4alpha-hydroxymethyl-stigmasta-7,24(241)-dien-3beta-ol-methyl oxidase activity [GO:0102180] (molecular function) Relationships: is a type of GO:0016709 Definition: Catalysis of the reaction: 4alpha-hydroxymethyl-stigmasta-7,24(241)-dien-3beta-ol + NADH + O2 + H+ = 4alpha-formyl-stigmasta-7,24(241)-dien-3beta-ol + NAD + 2 H2O. Sources: GOC:pz, RHEA:59036